ciliary base [GO:0097546] (cellular component) Definition: Area of the cilium (also called flagellum) where the basal body and the axoneme are anchored to the plasma membrane. The ciliary base encompasses the distal part of the basal body, transition fibers and transition zone and is structurally and functionally very distinct from the rest of the cilium. In this area proteins are sorted and filtered before entering the cilium, and many ciliary proteins localize specifically to this area. References: PMID:22653444 Sources: GOC:cilia, GOC:krc Note: Due to resolution issues, researchers are often unable to assign protein localization to more specific ciliary compartments such as the basal body, transition fibers or transition zone, and instead refer to 'ciliary base'. The terms GO:0036064 'ciliary basal body', GO:0097539 'ciliary transition fiber' and GO:0035869 'ciliary transition zone' represent strictly defined compartments at the ciliary base and should be used for annotation whenever possible. Also, note that cilia and eukaryotic flagella are deemed to be equivalent. Relationships: is a type of GO:0110165; is part of cilium [GO:0005929]; has part ciliary transition zone [GO:0035869]; BFO_0000051 GO:0097539 Also known as: cilial base, cilium base, flagellar base, flagellum base